{
  "gene": "UniProtKB:Q14943",
  "gene_symbol": "KIR3DS1",
  "term_label": "plasma membrane",
  "gene_name": "Killer cell immunoglobulin-like receptor 3DS1",
  "term_id": "GO:0005886"
}